{
  "gene_symbol": "ARHGAP12",
  "gene_name": "Rho GTPase-activating protein 12",
  "gene": "UniProtKB:Q8IWW6",
  "term_id": "GO:0005737",
  "term_label": "cytoplasm"
}